{
  "gene_name": "Syntaxin-10",
  "term_label": "SNAP receptor activity",
  "gene_symbol": "STX10",
  "gene": "UniProtKB:O60499",
  "term_id": "GO:0005484"
}